{
  "term_id": "UNKNOWN:0001",
  "gene": "UniProtKB:O95199",
  "gene_symbol": "RCBTB2",
  "term_label": "Unknown molecular function",
  "gene_name": "RCC1 and BTB domain-containing protein 2"
}